{
  "gene": "UniProtKB:Q14964",
  "gene_name": "Ras-related protein Rab-39A",
  "term_label": "GTPase activity",
  "gene_symbol": "RAB39A",
  "term_id": "GO:0003924"
}